juglone 3-hydroxylase activity [GO:0050012] (molecular function) Relationships: is a type of oxidoreductase activity, acting on CH or CH2 groups, oxygen as acceptor [GO:0016727] References: PMID:4041238 Sources: RHEA:18745 Definition: Catalysis of the reaction: 2 juglone + O2 = 2 3,5-dihydroxy-1,4-naphthoquinone + 2 H+. Also known as: juglone 3-monooxygenase activity, juglone hydroxylase activity, 5-hydroxy-1,4-naphthoquinone,hydrogen-donor:oxygen oxidoreductase (3-hydroxylating), naphthoquinone hydroxylase activity